positive regulation of macrophage migration [GO:1905523] (biological process) Relationships: is a type of positive regulation of mononuclear cell migration [GO:0071677]; is a type of regulation of macrophage migration [GO:1905521]; positively regulates macrophage migration [GO:1905517] References: PMID:25749876 Sources: GOC:TermGenie, GO_REF:0000058 Definition: Any process that activates or increases the frequency, rate or extent of macrophage migration. Also known as: up regulation of macrophage migration, up-regulation of macrophage migration, upregulation of macrophage migration, activation of macrophage migration Subtypes: GO:0010759, GO:1904141